arsenite methyltransferase activity [GO:0030791] (molecular function) Definition: Catalysis of the reaction: S-adenosyl-L-methionine + arsenite = S-adenosyl-L-homocysteine + methylarsonate. Sources: EC:2.1.1.137 Also known as: S-adenosyl-L-methionine:arsenic(III) methyltransferase activity, S-adenosyl-L-methionine:arsenite As-methyltransferase activity, S-adenosyl-L-methionine:methylarsonite As-methyltransferase activity Note: Note that the enzyme arsenite methyltransferase also has methylarsonite methyltransferase activity (GO:0030792). Relationships: is_a GO:0008757